endosome to lysosome transport [GO:0008333] (biological process) Subtypes: GO:0032510, endosome to lysosome transport of low-density lipoprotein particle [GO:0090117], neurotransmitter receptor transport, postsynaptic endosome to lysosome [GO:0098943] Definition: The directed movement of substances from endosomes to lysosomes. Sources: GOC:ai, ISBN:0716731363 Relationships: is a type of lysosomal transport [GO:0007041]; is a type of vesicle-mediated transport [GO:0016192]